{
  "term_id": "GO:0006825",
  "gene_symbol": "ATOX1",
  "gene": "UniProtKB:O00244",
  "gene_name": "Copper transport protein ATOX1",
  "term_label": "copper ion transport"
}